{
  "gene_symbol": "IGHD6-19",
  "gene_name": "Immunoglobulin heavy diversity 6-19 (Fragment)",
  "gene": "UniProtKB:A0A1Y8EKQ5",
  "term_label": "Unknown cellular component",
  "term_id": "UNKNOWN:0003"
}